{
  "gene_name": "Piercer of microtubule wall 1 protein",
  "term_label": "Unknown biological process",
  "gene_symbol": "PIERCE1",
  "term_id": "UNKNOWN:0002",
  "gene": "UniProtKB:Q5BN46"
}